{
  "gene": "UniProtKB:P01566",
  "term_id": "GO:0005132",
  "gene_symbol": "IFNA10",
  "term_label": "type I interferon receptor binding",
  "gene_name": "Interferon alpha-10"
}